{
  "gene": "UniProtKB:O95484",
  "term_id": "GO:0005923",
  "term_label": "bicellular tight junction",
  "gene_symbol": "CLDN9",
  "gene_name": "Claudin-9"
}